AAG codon-amino acid adaptor activity [GO:0033444] (molecular function) Note: Note that in the standard genetic code, AAG codes for lysine. Relationships: is a type of GO:0030533 Definition: A triplet codon-amino acid adaptor activity that recognizes an AAG codon. Sources: GOC:mah Also known as: lysine tRNA